positive regulation of regulation of vascular associated smooth muscle cell membrane depolarization [GO:1904199] (biological process) Relationships: is a type of positive regulation of membrane depolarization [GO:1904181]; positively regulates regulation of vascular associated smooth muscle cell membrane depolarization [GO:1990736] Definition: Any process that activates or increases the frequency, rate or extent of regulation of vascular smooth muscle cell membrane depolarization. References: PMID:20826763 Sources: GOC:TermGenie, GO_REF:0000058 Also known as: positive regulation of regulation of vascular smooth muscle cell membrane depolarization, up regulation of regulation of vascular smooth muscle cell membrane depolarization, up-regulation of regulation of vascular smooth muscle cell membrane depolarization, upregulation of regulation of vascular smooth muscle cell membrane depolarization, activation of regulation of vascular smooth muscle cell membrane depolarization